{
  "term_id": "GO:0003723",
  "gene": "UniProtKB:Q9BUJ2",
  "gene_name": "Heterogeneous nuclear ribonucleoprotein U-like protein 1",
  "term_label": "RNA binding",
  "gene_symbol": "HNRNPUL1"
}